regulation of cell proliferation involved in outflow tract morphogenesis [GO:1901963] (biological process) References: PMID:21419760 Sources: GOC:TermGenie, GOC:dph, GOC:mtg_heart Relationships: is a type of regulation of cell proliferation involved in heart morphogenesis [GO:2000136]; regulates cell proliferation involved in outflow tract morphogenesis [GO:0061325] Subtypes: positive regulation of cell proliferation involved in outflow tract morphogenesis [GO:1901964] Definition: Any process that modulates the frequency, rate or extent of cell proliferation involved in outflow tract morphogenesis.